{
  "term_label": "Unknown molecular function",
  "gene_name": "Inactive glutathione hydrolase 2",
  "term_id": "UNKNOWN:0001",
  "gene": "UniProtKB:P36268",
  "gene_symbol": "GGT2P"
}